{
  "gene_name": "Neurotrypsin",
  "gene_symbol": "PRSS12",
  "term_id": "GO:0030425",
  "term_label": "dendrite",
  "gene": "UniProtKB:P56730"
}